host intracellular membrane-bounded organelle [GO:0033648] (cellular component) Subtypes: host cell mitochondrion [GO:0033650], host cell plastid [GO:0033651], host cell nucleus [GO:0042025], host symbiosome [GO:0043658], host cell cytoplasmic vesicle [GO:0044161], host cell endoplasmic reticulum [GO:0044165], host cell endoplasmic reticulum-Golgi intermediate compartment [GO:0044172], host cell endosome [GO:0044174], host cell lysosome [GO:0044187], GO:0072517, GO:0120149 Relationships: is a type of host intracellular organelle [GO:0033647] Definition: Organized structure of distinctive morphology and function, as found in host cells, bounded by a single or double lipid bilayer membrane and occurring within the cell. Includes the nucleus, mitochondria, plastids, vacuoles, and vesicles. Excludes the plasma membrane. The host is defined as the larger of the organisms involved in a symbiotic interaction. Sources: GOC:pamgo_curators Also known as: host intracellular membrane-enclosed organelle